endo-alpha-N-acetylgalactosaminidase activity [GO:0033926] (molecular function) Relationships: is a type of GO:0004553; is a type of catalytic activity, acting on a glycoprotein [GO:0140103] Sources: EC:3.2.1.97 Also known as: mucinaminylserine mucinaminidase activity, D-galactosyl-3-(N-acetyl-alpha-D-galactosaminyl)-L-serine mucinaminohydrolase activity, D-galactosyl-N-acetyl-alpha-D-galactosamine D-galactosyl-N-acetyl-galactosaminohydrolase activity, endo-alpha-acetylgalactosaminidase activity Definition: Catalysis of the reactions : D-galactosyl-3-(N-acetyl-beta-D-galactosaminyl)-L-serine + H2O = D-galactosyl-3-N-acetyl-beta-D-galactosamine + L-serine and D-galactosyl-3-(N-acetyl-beta-D-galactosaminyl)-L-threonyl + H2O = D-galactosyl-3-N-acetyl-beta-D-galactosamine + L-threonyl.